{
  "term_label": "Unknown molecular function",
  "gene_symbol": "TRAJ23",
  "gene_name": "T cell receptor alpha joining 23 (Fragment)",
  "term_id": "UNKNOWN:0001",
  "gene": "UniProtKB:A0A075B6U7"
}